{
  "term_label": "proteolysis involved in protein catabolic process",
  "gene_symbol": "PSMB1",
  "gene": "UniProtKB:P20618",
  "term_id": "GO:0051603",
  "gene_name": "Proteasome subunit beta type-1"
}